{
  "term_id": "GO:0015485",
  "gene_name": "Steroidogenic acute regulatory protein, mitochondrial",
  "term_label": "cholesterol binding",
  "gene": "UniProtKB:P49675",
  "gene_symbol": "STAR"
}